{
  "gene": "UniProtKB:Q96KC2",
  "term_id": "GO:1903292",
  "gene_symbol": "ARL5B",
  "term_label": "protein localization to Golgi membrane",
  "gene_name": "ADP-ribosylation factor-like protein 5B"
}